{
  "gene_name": "Putative uncharacterized protein ADARB2-AS1",
  "term_id": "UNKNOWN:0002",
  "term_label": "Unknown biological process",
  "gene": "UniProtKB:A8MUL3",
  "gene_symbol": "ADARB2-AS1"
}